{
  "gene_name": "MAP_microtubule affinity-regulating kinase 3",
  "gene": "UniProtKB:P27448",
  "term_id": "GO:0000226",
  "term_label": "microtubule cytoskeleton organization",
  "gene_symbol": "MARK3"
}